{
  "term_label": "CBM complex",
  "gene_symbol": "BCL10",
  "gene_name": "B-cell lymphoma_leukemia 10",
  "gene": "UniProtKB:O95999",
  "term_id": "GO:0032449"
}